DNA-templated transcription termination [GO:0006353] (biological process) Definition: The completion of transcription: the RNA polymerase pauses, the RNA-DNA hybrid dissociates, followed by the release of the RNA polymerase from its DNA template. References: PMID:15020047, PMID:18280161, PMID:30978344 Sources: GOC:txnOH Also known as: transcriptional complex disassembly, DNA-dependent transcription, termination, DNA-templated transcription, termination, termination of DNA-dependent transcription, termination of transcription, DNA-dependent, transcription termination from bacterial-type RNA polymerase promoter, transcription termination factor activity, transcription termination, DNA-dependent Relationships: is a type of RNA biosynthetic process [GO:0032774]; is part of GO:0006351 Subtypes: termination of RNA polymerase I transcription [GO:0006363], termination of RNA polymerase II transcription [GO:0006369], termination of RNA polymerase III transcription [GO:0006386], termination of mitochondrial transcription [GO:0006393] Regulation: regulated by regulation of termination of DNA-templated transcription [GO:0031554]; positively regulated by positive regulation of termination of DNA-templated transcription [GO:0060566]; negatively regulated by negative regulation of termination of DNA-templated transcription [GO:0060567]